cyclin D1-CDK4 complex [GO:0097128] (cellular component) References: PMID:15935619 Sources: GOC:so Relationships: is a type of cyclin-dependent protein kinase holoenzyme complex [GO:0000307] Definition: A protein complex consisting of cyclin D1 and cyclin-dependent kinase 4 (CDK4). Cyclins are characterized by periodicity in protein abundance throughout the cell cycle. Cyclin-dependent kinases represent a family of serine/threonine protein kinases that become active upon binding to a cyclin regulatory partner.